{
  "term_label": "basal cortex",
  "gene": "UniProtKB:Q7Z460",
  "term_id": "GO:0045180",
  "gene_symbol": "CLASP1",
  "gene_name": "CLIP-associating protein 1"
}